negative regulation of macrophage proliferation [GO:0120042] (biological process) Definition: Any process that stops, prevents, or reduces the frequency, rate or extent of macrophage proliferation. Sources: GOC:BHF, GOC:BHF_miRNA, GOC:rph Relationships: is a type of negative regulation of leukocyte proliferation [GO:0070664]; is_a GO:0120040; negatively regulates macrophage proliferation [GO:0061517]